{
  "term_label": "nucleus",
  "term_id": "GO:0005634",
  "gene_symbol": "L3MBTL4",
  "gene_name": "Lethal(3)malignant brain tumor-like protein 4",
  "gene": "UniProtKB:Q8NA19"
}